{
  "gene_symbol": "ACOX2",
  "gene_name": "Peroxisomal acyl-coenzyme A oxidase 2",
  "gene": "UniProtKB:Q99424",
  "term_label": "fatty acid beta-oxidation using acyl-CoA oxidase",
  "term_id": "GO:0033540"
}